{
  "gene_symbol": "ZMYND10",
  "gene": "UniProtKB:O75800",
  "term_label": "cytoplasm",
  "term_id": "GO:0005737",
  "gene_name": "Zinc finger MYND domain-containing protein 10"
}